{
  "term_label": "cilium assembly",
  "gene_symbol": "DISC1",
  "term_id": "GO:0060271",
  "gene_name": "Disrupted in schizophrenia 1 protein",
  "gene": "UniProtKB:Q9NRI5"
}